{
  "gene": "UniProtKB:Q86SQ3",
  "gene_symbol": "ADGRE4P",
  "term_id": "GO:0004930",
  "term_label": "G protein-coupled receptor activity",
  "gene_name": "Putative adhesion G protein-coupled receptor E4P"
}